{
  "gene": "UniProtKB:P46782",
  "term_label": "ribosome",
  "gene_symbol": "RPS5",
  "gene_name": "Small ribosomal subunit protein uS7",
  "term_id": "GO:0005840"
}